{
  "term_label": "Cul2-RING ubiquitin ligase complex",
  "gene_name": "PRAME family member 10",
  "term_id": "GO:0031462",
  "gene": "UniProtKB:O60809",
  "gene_symbol": "PRAMEF10"
}